{
  "gene": "UniProtKB:P12838",
  "term_id": "GO:0061844",
  "gene_symbol": "DEFA4",
  "term_label": "antimicrobial humoral immune response mediated by antimicrobial peptide",
  "gene_name": "Defensin alpha 4"
}